{
  "gene_name": "Testis-expressed protein 46",
  "gene_symbol": "TEX46",
  "gene": "UniProtKB:H3BTG2",
  "term_id": "UNKNOWN:0003",
  "term_label": "Unknown cellular component"
}